{
  "gene_symbol": "H3Y2",
  "term_id": "GO:0007080",
  "gene_name": "Histone H3.X",
  "gene": "UniProtKB:P0DPK5",
  "term_label": "mitotic metaphase chromosome alignment"
}